regulation of cell shape [GO:0008360] (biological process) Sources: GOC:dph, GOC:go_curators, GOC:tb Relationships: is a type of regulation of cell morphogenesis [GO:0022604]; is a type of regulation of biological quality [GO:0065008] Definition: Any process that modulates the surface configuration of a cell. Subtypes: GO:0016476, regulation of direction of cell growth [GO:0061389], GO:0071963, regulation of establishment or maintenance of cell polarity regulating cell shape [GO:2000769]